{
  "term_id": "UNKNOWN:0003",
  "gene_symbol": "SUSD4",
  "gene": "UniProtKB:Q5VX71",
  "term_label": "Unknown cellular component",
  "gene_name": "Sushi domain-containing protein 4"
}